{
  "term_id": "GO:0061630",
  "gene": "UniProtKB:Q8TDB6",
  "gene_name": "E3 ubiquitin-protein ligase DTX3L",
  "gene_symbol": "DTX3L",
  "term_label": "ubiquitin protein ligase activity"
}